{
  "gene_symbol": "IL12B",
  "gene": "UniProtKB:P29460",
  "term_id": "GO:0042164",
  "term_label": "interleukin-12 alpha subunit binding",
  "gene_name": "Interleukin-12 subunit beta"
}